{
  "gene": "UniProtKB:A6NLJ0",
  "gene_symbol": "C2CD4B",
  "term_id": "UNKNOWN:0003",
  "gene_name": "C2 calcium-dependent domain-containing protein 4B",
  "term_label": "Unknown cellular component"
}